{
  "gene_symbol": "CHMP1A",
  "term_label": "protein transport",
  "term_id": "GO:0015031",
  "gene_name": "Charged multivesicular body protein 1a",
  "gene": "UniProtKB:Q9HD42"
}